{
  "gene": "UniProtKB:Q9UJ90",
  "term_id": "GO:1902282",
  "term_label": "voltage-gated potassium channel activity involved in ventricular cardiac muscle cell action potential repolarization",
  "gene_symbol": "KCNE5",
  "gene_name": "Potassium voltage-gated channel subfamily E regulatory beta subunit 5"
}